organ induction [GO:0001759] (biological process) Relationships: is a type of regulation of animal organ formation [GO:0003156]; is_a developmental induction [GO:0031128]; is a type of positive regulation of animal organ morphogenesis [GO:0110110]; positively regulates specification of animal organ identity [GO:0010092] Sources: ISBN:0878932437 Subtypes: heart induction [GO:0003129], lung induction [GO:0060492], prostate induction [GO:0060514], pancreas induction [GO:0061132] Also known as: induction of an organ Definition: The interaction of two or more cells or tissues that causes them to change their fates and specify the development of an organ.